BID-BCL-2 complex [GO:0097139] (cellular component) Relationships: is a type of Bcl-2 family protein complex [GO:0097136] References: PMID:14634621 Sources: GOC:so Definition: A heterodimeric protein complex consisting of BID and BCL-2, members of the Bcl-2 family of anti- and proapoptotic regulators.